{
  "term_id": "GO:0008017",
  "gene": "UniProtKB:A6NCE7",
  "gene_name": "Microtubule-associated proteins 1A_1B light chain 3 beta 2",
  "gene_symbol": "MAP1LC3B2",
  "term_label": "microtubule binding"
}